{
  "gene": "UniProtKB:O15438",
  "gene_symbol": "ABCC3",
  "term_id": "GO:0005886",
  "gene_name": "ATP-binding cassette sub-family C member 3",
  "term_label": "plasma membrane"
}